{
  "gene_symbol": "ZNF730",
  "term_label": "RNA polymerase II cis-regulatory region sequence-specific DNA binding",
  "term_id": "GO:0000978",
  "gene_name": "Putative zinc finger protein 730",
  "gene": "UniProtKB:Q6ZMV8"
}